geranylgeranyl diphosphate reductase activity [GO:0102067] (molecular function) Relationships: is a type of oxidoreductase activity, acting on the CH-CH group of donors, NAD or NADP as acceptor [GO:0016628] Definition: Catalysis of the reaction: (E)-3,7,11,15-tetramethylhexadec-2-en-1-yl diphosphate + 3 NADP = 2-trans,6-trans,10-trans-geranylgeranyl diphosphate + 3 NADPH + 3 H+. Sources: EC:1.3.1.83, GOC:pz